{
  "term_id": "GO:0005634",
  "gene_name": "Histone H2B type 1-J",
  "gene": "UniProtKB:P06899",
  "gene_symbol": "H2BC11",
  "term_label": "nucleus"
}